phytoalexin catabolic process [GO:0052316] (biological process) Also known as: phytoalexin catabolism Sources: GOC:ai Subtypes: indole phytoalexin catabolic process [GO:0046216], flavonoid phytoalexin catabolic process [GO:0046286], isoflavonoid phytoalexin catabolic process [GO:0046290] Relationships: is a type of toxin catabolic process [GO:0009407]; is a type of phytoalexin metabolic process [GO:0052314] Definition: The chemical reactions and pathways resulting in the breakdown of phytoalexins, any of a range of substances produced by plants as part of their defense response.